{
  "term_id": "UNKNOWN:0001",
  "gene_symbol": "FRMD3",
  "gene_name": "FERM domain-containing protein 3",
  "term_label": "Unknown molecular function",
  "gene": "UniProtKB:A2A2Y4"
}